{
  "term_id": "GO:0050919",
  "gene_symbol": "SEMA4F",
  "gene_name": "Semaphorin-4F",
  "gene": "UniProtKB:O95754",
  "term_label": "negative chemotaxis"
}